mitochondrion localization [GO:0051646] (biological process) Relationships: is a type of organelle localization [GO:0051640] Also known as: establishment and maintenance of mitochondria localization, establishment and maintenance of mitochondrion localization, localization of mitochondria, localization of mitochondrion, mitochondria localization, mitochondrial localization, mitochondrion localisation Sources: GOC:ai Definition: Any process in which a mitochondrion or mitochondria are transported to, and/or maintained in, a specific location within the cell. Subtypes: mitochondrion distribution [GO:0048311], establishment of mitochondrion localization [GO:0051654], GO:0051659